{
  "gene_symbol": "ZNF414",
  "term_label": "Unknown cellular component",
  "term_id": "UNKNOWN:0003",
  "gene_name": "Zinc finger protein 414",
  "gene": "UniProtKB:Q96IQ9"
}